{
  "term_label": "signaling receptor binding",
  "gene_name": "Lymphocyte function-associated antigen 3",
  "term_id": "GO:0005102",
  "gene_symbol": "CD58",
  "gene": "UniProtKB:P19256"
}